{
  "gene_name": "GTP-binding protein RAD",
  "term_id": "UNKNOWN:0002",
  "gene_symbol": "RRAD",
  "gene": "UniProtKB:P55042",
  "term_label": "Unknown biological process"
}